{
  "gene": "UniProtKB:Q9UQ03",
  "term_id": "GO:0051015",
  "gene_name": "Coronin-2B",
  "term_label": "actin filament binding",
  "gene_symbol": "CORO2B"
}